{
  "term_id": "GO:0071482",
  "gene": "UniProtKB:Q9H1Y3",
  "term_label": "cellular response to light stimulus",
  "gene_name": "Opsin-3",
  "gene_symbol": "OPN3"
}